4-sulfobenzoate 3,4-dioxygenase activity [GO:0018621] (molecular function) Relationships: is a type of oxidoreductase activity, acting on paired donors, with incorporation or reduction of molecular oxygen, NAD(P)H as one donor, and incorporation of two atoms of oxygen into one donor [GO:0016708] Definition: Catalysis of the reaction: 4-sulfobenzoate + H+ + NADH + O2 = 3,4-dihydroxybenzoate + NAD+ + sulfite. Sources: EC:1.14.12.8, RHEA:13937 Also known as: 4-sulphobenzoate 3,4-dioxygenase activity, 4-sulfobenzoate 3,4-dioxygenase system, 4-sulfobenzoate dioxygenase activity, 4-sulfobenzoate,NADH:oxygen oxidoreductase (3,4-hydroxylating, sulfite-forming)